{
  "gene": "UniProtKB:P50479",
  "gene_name": "PDZ and LIM domain protein 4",
  "gene_symbol": "PDLIM4",
  "term_label": "adherens junction",
  "term_id": "GO:0005912"
}